{
  "gene_name": "Ectonucleotide pyrophosphatase_phosphodiesterase family member 1",
  "term_id": "GO:0004528",
  "gene_symbol": "ENPP1",
  "term_label": "phosphodiesterase I activity",
  "gene": "UniProtKB:P22413"
}